{
  "gene_name": "Probable ribonuclease ZC3H12D",
  "term_id": "GO:0036464",
  "gene": "UniProtKB:A2A288",
  "gene_symbol": "ZC3H12D",
  "term_label": "cytoplasmic ribonucleoprotein granule"
}